{
  "term_id": "GO:0005737",
  "gene_symbol": "CSNK2B",
  "gene": "UniProtKB:P67870",
  "gene_name": "Casein kinase II subunit beta",
  "term_label": "cytoplasm"
}